{
  "term_label": "RNA polymerase II cis-regulatory region sequence-specific DNA binding",
  "term_id": "GO:0000978",
  "gene": "UniProtKB:O15178",
  "gene_symbol": "TBXT",
  "gene_name": "T-box transcription factor T"
}